{
  "gene_name": "cGMP-dependent 3',5'-cyclic phosphodiesterase",
  "gene": "UniProtKB:O00408",
  "gene_symbol": "PDE2A",
  "term_label": "cytosol",
  "term_id": "GO:0005829"
}